{
  "gene_name": "Zinc finger and BTB domain-containing protein 6",
  "term_label": "regulation of immune system process",
  "gene": "UniProtKB:Q15916",
  "gene_symbol": "ZBTB6",
  "term_id": "GO:0002682"
}